{
  "gene": "UniProtKB:Q9Y2A7",
  "term_label": "neuron projection morphogenesis",
  "gene_name": "Nck-associated protein 1",
  "term_id": "GO:0048812",
  "gene_symbol": "NCKAP1"
}